regulation of 1-phosphatidyl-1D-myo-inositol 4,5-bisphosphate catabolic process [GO:1902641] (biological process) Relationships: is a type of regulation of phospholipid catabolic process [GO:0060696]; regulates 1-phosphatidyl-1D-myo-inositol 4,5-bisphosphate catabolic process [GO:1902634] Also known as: regulation of 1-phosphatidyl-1D-myo-inositol 4,5-bisphosphate breakdown, regulation of 1-phosphatidyl-1D-myo-inositol 4,5-bisphosphate catabolism, regulation of 1-phosphatidyl-1D-myo-inositol 4,5-bisphosphate degradation References: PMID:22562153 Sources: GOC:TermGenie, GOC:di, GO_REF:0000058 Definition: Any process that modulates the frequency, rate or extent of 1-phosphatidyl-1D-myo-inositol 4,5-bisphosphate catabolic process. Subtypes: negative regulation of 1-phosphatidyl-1D-myo-inositol 4,5-bisphosphate catabolic process [GO:1902642], positive regulation of 1-phosphatidyl-1D-myo-inositol 4,5-bisphosphate catabolic process [GO:1902643]